{
  "gene_name": "Trace amine-associated receptor 5",
  "term_id": "GO:0001594",
  "term_label": "trace-amine receptor activity",
  "gene": "UniProtKB:O14804",
  "gene_symbol": "TAAR5"
}